SH3 domain binding [GO:0017124] (molecular function) Relationships: is a type of protein domain specific binding [GO:0019904] Sources: GOC:go_curators, Pfam:PF00018 Definition: Binding to a SH3 domain (Src homology 3) of a protein, small protein modules containing approximately 50 amino acid residues found in a great variety of intracellular or membrane-associated proteins.